microtubule bundle formation [GO:0001578] (biological process) Definition: A process that results in a parallel arrangement of microtubules. Relationships: is a type of GO:0000226 Subtypes: axoneme assembly [GO:0035082], microtubule bundle formation involved in mitotic spindle midzone assembly [GO:1903562], microtubule bundle formation involved in horsetail-astral microtubule organization [GO:1903563] Sources: GOC:dph Also known as: microtubule bundling